nucleosomal methylation activator complex [GO:0070311] (cellular component) Also known as: NUMAC Relationships: is a type of GO:0035097 References: PMID:14729568 Sources: GOC:mah Definition: A protein complex that contains eight subunits in common with the SWI/SNF complex, plus the ATPase BRG1 (SMARCA4) and the histone methyltransferase CARM1; the complex is involved in regulating nuclear receptor-dependent transcription.